N-terminal peptidyl-methionine acetylation [GO:0017196] (biological process) Relationships: is a type of GO:0006474; is a type of GO:0018206 Regulation: regulated by GO:1904663; negatively regulated by GO:1904664; positively regulated by GO:1904665 Definition: The acetylation of the N-terminal methionine of proteins to form the derivative N-acetyl-L-methionine. Sources: RESID:AA0049